{
  "term_label": "lipid storage",
  "gene_symbol": "FITM2",
  "gene": "UniProtKB:Q8N6M3",
  "term_id": "GO:0019915",
  "gene_name": "Acyl-coenzyme A diphosphatase FITM2"
}